{
  "term_id": "GO:0005737",
  "gene": "UniProtKB:Q8TF09",
  "gene_name": "Dynein light chain roadblock-type 2",
  "term_label": "cytoplasm",
  "gene_symbol": "DYNLRB2"
}